collagen type IX trimer [GO:0005594] (CC) References: PMID:21421911 Relationships: is a type of GO:0005593 Definition: A collagen heterotrimer containing type IX alpha chains in alpha1(IX)alpha2(IX)alpha3(IX) trimers; type IX collagen triple helices associate to form a structure that links glycosaminoglycans to type II collagen fibrils.